negative regulation of dopamine metabolic process [GO:0045963] (biological process) Sources: GOC:go_curators Also known as: down regulation of dopamine metabolic process, down-regulation of dopamine metabolic process, downregulation of dopamine metabolic process, negative regulation of dopamine metabolism, inhibition of dopamine metabolic process Definition: Any process that stops, prevents, or reduces the frequency, rate or extent of the chemical reactions and pathways involving dopamine. Relationships: is a type of negative regulation of amine metabolic process [GO:0033239]; is a type of regulation of dopamine metabolic process [GO:0042053]; negatively regulates GO:0042417 Subtypes: negative regulation of dopamine biosynthetic process [GO:1903180]